{
  "gene_symbol": "IFT57",
  "term_label": "non-motile cilium assembly",
  "term_id": "GO:1905515",
  "gene": "UniProtKB:Q9NWB7",
  "gene_name": "Intraflagellar transport protein 57 homolog"
}